{
  "gene_name": "Allograft inflammatory factor 1",
  "gene_symbol": "AIF1",
  "term_label": "actin filament",
  "term_id": "GO:0005884",
  "gene": "UniProtKB:P55008"
}